{
  "gene_symbol": "RPL7",
  "term_id": "GO:0022625",
  "gene_name": "Large ribosomal subunit protein uL30",
  "term_label": "cytosolic large ribosomal subunit",
  "gene": "UniProtKB:P18124"
}